negative regulation of telomeric loop disassembly [GO:1904534] (biological process) Definition: Any process that stops, prevents or reduces the frequency, rate or extent of telomeric loop disassembly. References: PMID:22579284 Sources: GOC:BHF, GOC:BHF_telomere, GOC:TermGenie, GOC:nc, GO_REF:0000058 Also known as: down regulation of T loop disassembly, down regulation of telomeric loop disassembly, down-regulation of T loop disassembly, down-regulation of telomeric loop disassembly, downregulation of T loop disassembly, downregulation of telomeric loop disassembly, negative regulation of T loop disassembly, inhibition of T loop disassembly, inhibition of telomeric loop disassembly Subtypes: GO:1905839 Relationships: is a type of negative regulation of telomere maintenance [GO:0032205]; is a type of regulation of telomeric loop disassembly [GO:1904533]; negatively regulates telomeric loop disassembly [GO:0090657]